{
  "gene_symbol": "PPP1R12C",
  "term_id": "GO:0048812",
  "gene_name": "Protein phosphatase 1 regulatory subunit 12C",
  "gene": "UniProtKB:Q9BZL4",
  "term_label": "neuron projection morphogenesis"
}